{
  "gene_symbol": "STX4",
  "term_label": "vesicle docking",
  "gene": "UniProtKB:Q12846",
  "term_id": "GO:0048278",
  "gene_name": "Syntaxin-4"
}